magnesium-dependent protein serine/threonine phosphatase complex [GO:0005963] (CC) Definition: An intracellular enzyme complex that catalyzes the removal of serine- or threonine-bound phosphate groups from a wide range of phosphoproteins, including a number of enzymes that have been phosphorylated under the action of a kinase. References: PMID:17517611, PMID:22343722 Relationships: is a type of protein serine/threonine phosphatase complex [GO:0008287]; is a type of intracellular protein-containing complex [GO:0140535]